{
  "term_label": "GTPase activity",
  "gene_name": "GTP-binding protein Rheb",
  "term_id": "GO:0003924",
  "gene": "UniProtKB:Q15382",
  "gene_symbol": "RHEB"
}